G protein-coupled cytokinin receptor activity [GO:0001647] (molecular function) Relationships: is a type of G protein-coupled receptor activity [GO:0004930]; is a type of cytokinin receptor activity [GO:0009884] Also known as: G protein coupled cytokinin receptor activity, G-protein coupled cytokinin receptor activity, cytokinin receptor activity, G-protein coupled Definition: Combining with cytokinin and transmitting the signal across the membrane by activating an associated G-protein; promotes the exchange of GDP for GTP on the alpha subunit of a heterotrimeric G-protein complex. Sources: GOC:bf, GOC:dph